{
  "gene_symbol": "HIF1AN",
  "term_id": "GO:0036139",
  "term_label": "peptidyl-histidine dioxygenase activity",
  "gene": "UniProtKB:Q9NWT6",
  "gene_name": "Hypoxia-inducible factor 1-alpha inhibitor"
}